L-aspartate transmembrane transport [GO:0070778] (biological process) References: PMID:21307582 Also known as: L-aspartate transport Definition: The directed movement of L-aspartate across a membrane by means of some agent such as a transporter or a pore. Relationships: is a type of aspartate transmembrane transport [GO:0015810]; is a type of GO:1902475 Subtypes: L-aspartate transmembrane export from vacuole [GO:0089703], L-aspartate import across plasma membrane [GO:0140009]